negative regulation of lung alveolus development [GO:1904654] (biological process) Definition: Any process that stops, prevents or reduces the frequency, rate or extent of lung alveolus development. Also known as: down regulation of alveolarization, down regulation of alveologenesis, down regulation of lung alveolus development, down-regulation of alveolarization, down-regulation of alveologenesis, down-regulation of lung alveolus development, downregulation of alveolarization, downregulation of alveologenesis, downregulation of lung alveolus development, negative regulation of alveolarization, negative regulation of alveologenesis, inhibition of alveolarization, inhibition of alveologenesis, inhibition of lung alveolus development References: PMID:23962064 Sources: GOC:TermGenie, GO_REF:0000058 Relationships: is a type of negative regulation of developmental process [GO:0051093]; is a type of negative regulation of multicellular organismal process [GO:0051241]; is a type of regulation of lung alveolus development [GO:1904653]; negatively regulates lung alveolus development [GO:0048286]